{
  "gene_symbol": "TIMM23B",
  "gene_name": "Mitochondrial import inner membrane translocase subunit Tim23B",
  "term_id": "GO:0005744",
  "term_label": "TIM23 mitochondrial import inner membrane translocase complex",
  "gene": "UniProtKB:Q5SRD1"
}